{
  "term_id": "GO:0005886",
  "gene": "UniProtKB:Q9NPD7",
  "gene_symbol": "NRN1",
  "term_label": "plasma membrane",
  "gene_name": "Neuritin"
}